negative regulation of mitochondrial ATP synthesis coupled proton transport [GO:1905707] (biological process) Definition: Any process that stops, prevents or reduces the frequency, rate or extent of mitochondrial ATP synthesis coupled proton transport. Relationships: is a type of regulation of mitochondrial ATP synthesis coupled proton transport [GO:1905706]; is a type of GO:2001170; negatively regulates GO:0042776 References: PMID:12809520, PMID:15294286 Sources: GOC:TermGenie, GO_REF:0000058